{
  "term_label": "endosome",
  "gene_symbol": "MYCBPAP",
  "gene": "UniProtKB:Q8TBZ2",
  "term_id": "GO:0005768",
  "gene_name": "MYCBP-associated protein"
}